{
  "term_id": "UNKNOWN:0001",
  "term_label": "Unknown molecular function",
  "gene_symbol": "POTEH",
  "gene_name": "POTE ankyrin domain family member H",
  "gene": "UniProtKB:Q6S545"
}